{
  "gene_symbol": "IL6ST",
  "term_id": "GO:0019981",
  "gene": "UniProtKB:P40189",
  "gene_name": "Interleukin-6 receptor subunit beta",
  "term_label": "interleukin-6 binding"
}